negative regulation of erythrocyte enucleation [GO:0061932] (biological process) Relationships: is a type of GO:0051129; is a type of regulation of erythrocyte enucleation [GO:0061930]; is a type of negative regulation of cell maturation [GO:1903430]; negatively regulates erythrocyte enucleation [GO:0043131] References: PMID:25241935 Definition: Any process that decreases the frequency, rate or extent of erythrocyte enucleation.